regulation of polyamine biosynthetic process [GO:0010967] (biological process) Sources: GOC:dph, GOC:tb Definition: Any process that modulates the frequency, rate or extent of polyamine biosynthesis. Polyamine biosynthesis is the chemical reactions and pathways resulting in the formation of polyamines, any organic compound containing two or more amino groups. Relationships: is a type of regulation of biosynthetic process [GO:0009889]; is a type of regulation of amine metabolic process [GO:0033238]; is a type of regulation of primary metabolic process [GO:0080090]; RO_0002211 polyamine biosynthetic process [GO:0006596] Subtypes: negative regulation of polyamine biosynthetic process [GO:0170066], regulation of spermidine biosynthetic process [GO:1901304]